{
  "term_label": "kainate selective glutamate receptor activity",
  "gene": "UniProtKB:Q13003",
  "term_id": "GO:0015277",
  "gene_name": "Glutamate receptor ionotropic, kainate 3",
  "gene_symbol": "GRIK3"
}